psoralen synthase (NADPH) activity [GO:0102876] (molecular function) Definition: Catalysis of the reaction: (+)-marmesin + NADPH + H+ + O2 = psoralen + NADP + acetone + 2 H2O. Sources: EC:1.14.14.141 Relationships: is a type of oxidoreductase activity, acting on paired donors, with incorporation or reduction of molecular oxygen, NAD(P)H as one donor, and incorporation of one atom of oxygen [GO:0016709]